{
  "term_label": "plasma membrane",
  "gene": "UniProtKB:Q07075",
  "gene_name": "Glutamyl aminopeptidase",
  "term_id": "GO:0005886",
  "gene_symbol": "ENPEP"
}